{
  "gene_name": "Lebercilin",
  "term_id": "GO:0042073",
  "gene_symbol": "LCA5",
  "gene": "UniProtKB:Q86VQ0",
  "term_label": "intraciliary transport"
}